{
  "gene": "UniProtKB:O15178",
  "term_label": "DNA-binding transcription factor activity, RNA polymerase II-specific",
  "term_id": "GO:0000981",
  "gene_symbol": "TBXT",
  "gene_name": "T-box transcription factor T"
}